negative regulation of maintenance of mitotic sister chromatid cohesion, arms [GO:2000716] (biological process) Definition: Any process that stops, prevents or reduces the frequency, rate or extent of maintenance of mitotic sister chromatid cohesion along the chromosome arms. Sources: GOC:mah Also known as: negative regulation of maintenance of mitotic sister chromatin cohesion along arms, negative regulation of maintenance of sister chromatin cohesion along arms at mitosis Relationships: is a type of negative regulation of maintenance of mitotic sister chromatid cohesion [GO:0034183]; is a type of regulation of maintenance of mitotic sister chromatid cohesion, arms [GO:2000715]; negatively regulates maintenance of mitotic sister chromatid cohesion, arms [GO:0071959]